trans-synaptic signaling by endocannabinoid, modulating synaptic transmission [GO:0099553] (biological process) Definition: Cell-cell signaling between presynapse and postsynapse, via the release and reception of endocannabinoid ligands, that modulates the synaptic transmission properties of the synapse. References: PMID:21531987 Sources: GOC:dos Note: Note that this term was created for the SynGO project, and will be obsoleted when the SynGO annotations are made in Noctua. Relationships: is_a trans-synaptic signaling by endocannabinoid [GO:0099542]; is a type of GO:0099552 Regulation: regulated by regulation of trans-synaptic signaling by endocannabinoid, modulating synaptic transmission [GO:0150036]